{
  "gene_symbol": "ZNF257",
  "gene": "UniProtKB:Q9Y2Q1",
  "term_label": "regulation of DNA-templated transcription",
  "term_id": "GO:0006355",
  "gene_name": "Zinc finger protein 257"
}